venom-mediated hemorrhage [GO:0044358] (biological process) Relationships: is a type of venom-mediated perturbation of hemostasis [GO:0044483] References: PMID:10441379, PMID:20614020 Also known as: envenomation resulting in hemorrhagic damage in another organism, envenomation resulting in hemorrhagic damage to other organism, venom-mediated hemorrhagic damage in another organism Definition: A process in which an organism causes vascular damage and hemorrhage in another organism via the action of a venom.